{
  "term_id": "GO:0019911",
  "gene": "UniProtKB:Q9Y342",
  "gene_symbol": "PLLP",
  "gene_name": "Plasmolipin",
  "term_label": "structural constituent of myelin sheath"
}